{
  "gene_symbol": "GTPBP6",
  "term_label": "Unknown biological process",
  "gene": "UniProtKB:O43824",
  "term_id": "UNKNOWN:0002",
  "gene_name": "Putative GTP-binding protein 6"
}